{
  "gene_name": "Immunoglobulin kappa joining 5 (Fragment)",
  "term_label": "Unknown biological process",
  "term_id": "UNKNOWN:0002",
  "gene_symbol": "IGKJ5",
  "gene": "UniProtKB:A0A0A0MTA3"
}